{
  "term_label": "DNA-binding transcription factor activity, RNA polymerase II-specific",
  "gene_symbol": "HOXA13",
  "gene_name": "Homeobox protein Hox-A13",
  "term_id": "GO:0000981",
  "gene": "UniProtKB:P31271"
}